{
  "gene_symbol": "SENP2",
  "term_label": "nucleus",
  "gene": "UniProtKB:Q9HC62",
  "term_id": "GO:0005634",
  "gene_name": "Sentrin-specific protease 2"
}